{
  "gene": "UniProtKB:O15457",
  "term_id": "GO:0007131",
  "term_label": "reciprocal meiotic recombination",
  "gene_name": "MutS protein homolog 4",
  "gene_symbol": "MSH4"
}